{
  "term_id": "GO:0000981",
  "gene": "UniProtKB:A6NJL1",
  "gene_symbol": "ZSCAN5B",
  "term_label": "DNA-binding transcription factor activity, RNA polymerase II-specific",
  "gene_name": "Zinc finger and SCAN domain-containing protein 5B"
}